G-protein gated potassium channel activity involved in regulation of postsynaptic membrane potential [GO:0099102] (molecular function) Definition: Any G-protein gated potassium channel activity that is involved regulation of postsynaptic membrane potential. References: PMID:9429760 Sources: GOC:dos Relationships: is a type of GO:0099101; is part of regulation of postsynaptic membrane potential [GO:0060078]